dendritic growth cone [GO:0044294] (cellular component) Definition: The migrating motile tip of a growing nerve cell dendrite. Relationships: is a type of growth cone [GO:0030426]; is a type of dendrite terminus [GO:0044292] Also known as: dendrite growth cone Sources: GOC:jl